{
  "gene_name": "E3 ubiquitin-protein ligase Praja-2",
  "term_label": "protein ubiquitination",
  "gene": "UniProtKB:O43164",
  "gene_symbol": "PJA2",
  "term_id": "GO:0016567"
}